{
  "term_label": "dynein intermediate chain binding",
  "gene_name": "Dynein light chain Tctex-type 5",
  "term_id": "GO:0045505",
  "gene": "UniProtKB:Q8N7M0",
  "gene_symbol": "DYNLT5"
}